{
  "gene": "UniProtKB:P09466",
  "gene_symbol": "PAEP",
  "term_id": "UNKNOWN:0002",
  "term_label": "Unknown biological process",
  "gene_name": "Glycodelin"
}